{
  "gene_name": "MHC class II regulatory factor RFX1",
  "term_label": "regulation of transcription by RNA polymerase II",
  "gene": "UniProtKB:P22670",
  "gene_symbol": "RFX1",
  "term_id": "GO:0006357"
}